{
  "gene_name": "PIH1 domain-containing protein 2",
  "gene": "UniProtKB:Q8WWB5",
  "term_id": "GO:0000492",
  "gene_symbol": "PIH1D2",
  "term_label": "box C/D snoRNP assembly"
}